protein-DNA complex disassembly [GO:0032986] (biological process) Sources: GOC:mah Definition: The disaggregation of a protein-DNA complex into its constituent components. Subtypes: nucleosome disassembly [GO:0006337], DNA recombinase disassembly [GO:1990986] Relationships: is a type of GO:0032984; is a type of protein-DNA complex organization [GO:0071824] Also known as: DNA-protein complex disassembly